ectoderm and mesoderm interaction [GO:0007499] (biological process) Also known as: ectoderm/mesoderm interaction Definition: A cell-cell signaling process occurring between the two gastrulation-generated layers of the ectoderm and the mesoderm. Relationships: is a type of cell-cell signaling [GO:0007267]; is part of mesoderm development [GO:0007498] Sources: GOC:isa_complete